trans-2-enoyl-CoA reductase (NADPH) activity [GO:0019166] (molecular function) Also known as: NADPH-dependent trans-2-enoyl-CoA reductase activity, acyl-CoA:NADP+ trans-2-oxidoreductase activity, reductase, trans-enoyl coenzyme A Definition: Catalysis of the reaction: acyl-CoA + NADP+ = trans-2,3-dehydroacyl-CoA + NADPH + H+. Relationships: is_a oxidoreductase activity, acting on the CH-CH group of donors, NAD or NADP as acceptor [GO:0016628] Sources: EC:1.3.1.38